{
  "term_id": "GO:0005794",
  "gene_symbol": "AOC3",
  "gene_name": "Membrane primary amine oxidase",
  "gene": "UniProtKB:Q16853",
  "term_label": "Golgi apparatus"
}